{
  "gene_symbol": "RPLP1",
  "gene_name": "Large ribosomal subunit protein P1",
  "term_id": "GO:0002181",
  "term_label": "cytoplasmic translation",
  "gene": "UniProtKB:P05386"
}